{
  "gene_symbol": "COL24A1",
  "gene_name": "Collagen alpha-1(XXIV) chain",
  "term_label": "basement membrane",
  "term_id": "GO:0005604",
  "gene": "UniProtKB:Q17RW2"
}